positive regulation of tumor necrosis factor superfamily cytokine production [GO:1903557] (BP) References: PMID:24187568 Sources: GOC:TermGenie, GO_REF:0000058 Also known as: positive regulation of TNFSF cytokine production, up regulation of TNFSF cytokine production, up regulation of tumor necrosis factor superfamily cytokine production, up-regulation of TNFSF cytokine production, up-regulation of tumor necrosis factor superfamily cytokine production, upregulation of TNFSF cytokine production, upregulation of tumor necrosis factor superfamily cytokine production, activation of TNFSF cytokine production, activation of tumor necrosis factor superfamily cytokine production, activation of TNF superfamily production, positive regulation of TNF superfamily production, up regulation of TNF superfamily production, up-regulation of TNF superfamily production, upregulation of TNF superfamily production Definition: Any process that activates or increases the frequency, rate or extent of tumor necrosis factor superfamily cytokine production. Subtypes: positive regulation of TRAIL production [GO:0032759], GO:0032760, positive regulation of lymphotoxin A production [GO:0032761], positive regulation of tumor necrosis factor (ligand) superfamily member 11 production [GO:2000309] Relationships: is a type of GO:0001819; is a type of regulation of tumor necrosis factor superfamily cytokine production [GO:1903555]; positively regulates GO:0071706